{
  "term_id": "GO:0003697",
  "gene": "UniProtKB:O95551",
  "gene_symbol": "TDP2",
  "gene_name": "Tyrosyl-DNA phosphodiesterase 2",
  "term_label": "single-stranded DNA binding"
}